{
  "gene": "UniProtKB:O60739",
  "term_label": "RNA binding",
  "term_id": "GO:0003723",
  "gene_name": "Eukaryotic translation initiation factor 1b",
  "gene_symbol": "EIF1B"
}